{
  "term_id": "GO:0005242",
  "term_label": "inward rectifier potassium channel activity",
  "gene_name": "ATP-sensitive inward rectifier potassium channel 14",
  "gene_symbol": "KCNJ14",
  "gene": "UniProtKB:Q9UNX9"
}